{
  "gene_symbol": "REM1",
  "term_id": "UNKNOWN:0002",
  "gene_name": "GTP-binding protein REM 1",
  "gene": "UniProtKB:O75628",
  "term_label": "Unknown biological process"
}